methyl jasmonate methylesterase activity [GO:0030795] (molecular function) Relationships: is a type of S-adenosylmethionine-dependent methyltransferase activity [GO:0008757] Sources: RHEA:13349 Also known as: S-adenosyl-L-methionine:jasmonic acid carboxyl methyltransferase activity, S-adenosyl-L-methionine:jasmonate O-methyltransferase activity, jasmonic acid carboxyl methyltransferase activity Definition: Catalysis of the reaction: S-adenosyl-L-methionine + a jasmonate = S-adenosyl-L-homocysteine + a methyljasmonate.